{
  "term_id": "GO:0055088",
  "gene": "UniProtKB:Q86TW2",
  "gene_name": "AarF domain-containing protein kinase 1",
  "term_label": "lipid homeostasis",
  "gene_symbol": "ADCK1"
}